{
  "gene_name": "E3 ubiquitin-protein ligase RNF19A",
  "gene_symbol": "RNF19A",
  "gene": "UniProtKB:Q9NV58",
  "term_label": "ubiquitin conjugating enzyme binding",
  "term_id": "GO:0031624"
}